L-arginine transmembrane transport from lysosomal lumen to cytosol [GO:1904917] (biological process) Relationships: is a type of transmembrane transport from lysosomal lumen to cytosol [GO:0170063]; is a type of L-arginine transmembrane export from vacuole [GO:1990818] Also known as: transmembrane L-arginine transport from lysosomal lumen to cytosol References: PMID:22822152 Sources: GOC:TermGenie, GOC:kmv, GO_REF:0000078 Definition: The directed movement of L-arginine across a membrane from lysosomal lumen to cytosol.